{
  "term_id": "GO:0019221",
  "term_label": "cytokine-mediated signaling pathway",
  "gene": "UniProtKB:P48357",
  "gene_name": "Leptin receptor",
  "gene_symbol": "LEPR"
}